{
  "gene_name": "Putative uncharacterized protein encoded by BRWD1-AS2",
  "term_label": "Unknown cellular component",
  "gene_symbol": "BRWD1-AS2",
  "gene": "UniProtKB:P59051",
  "term_id": "UNKNOWN:0003"
}